positive regulation of acinar cell proliferation [GO:1904699] (biological process) Also known as: positive regulation of acinic cell proliferation, positive regulation of acinous cell proliferation, up regulation of acinar cell proliferation, up regulation of acinic cell proliferation, up regulation of acinous cell proliferation, up-regulation of acinar cell proliferation, up-regulation of acinic cell proliferation, up-regulation of acinous cell proliferation, upregulation of acinar cell proliferation, upregulation of acinic cell proliferation, upregulation of acinous cell proliferation, activation of acinar cell proliferation, activation of acinic cell proliferation, activation of acinous cell proliferation References: PMID:9788538 Sources: GOC:TermGenie, GO_REF:0000058 Definition: Any process that activates or increases the frequency, rate or extent of acinar cell proliferation. Relationships: is a type of positive regulation of epithelial cell proliferation [GO:0050679]; is a type of regulation of acinar cell proliferation [GO:1904697]; positively regulates acinar cell proliferation [GO:1990863]